{
  "term_id": "UNKNOWN:0003",
  "gene_symbol": "PSG6",
  "gene_name": "Pregnancy-specific beta-1-glycoprotein 6",
  "gene": "UniProtKB:Q00889",
  "term_label": "Unknown cellular component"
}